phenylalanine decarboxylase activity [GO:0050174] (molecular function) Relationships: is a type of carboxy-lyase activity [GO:0016831] Also known as: aromatic L-amino acid decarboxylase activity, L-phenylalanine carboxy-lyase (phenylethylamine-forming), L-phenylalanine carboxy-lyase activity, L-phenylalanine decarboxylase activity Definition: Catalysis of the reaction: L-phenylalanine = phenylethylamine + CO2. Sources: EC:4.1.1.53, MetaCyc:PHENYLALANINE-DECARBOXYLASE-RXN